regulation of butyryl-CoA biosynthetic process from acetyl-CoA [GO:1900494] (biological process) Subtypes: negative regulation of butyryl-CoA biosynthetic process from acetyl-CoA [GO:1900495], positive regulation of butyryl-CoA biosynthetic process from acetyl-CoA [GO:1900496] Also known as: regulation of butyryl-CoA biosynthesis from acetyl-CoA Definition: Any process that modulates the frequency, rate or extent of butyryl-CoA biosynthetic process from acetyl-CoA. Sources: GOC:TermGenie, GOC:mengo_curators Relationships: is a type of regulation of fatty acid biosynthetic process [GO:0042304]; is a type of regulation of acyl-CoA biosynthetic process [GO:0050812]; RO_0002211 GO:0044579